{
  "gene_symbol": "EDDM3B",
  "term_label": "Unknown molecular function",
  "term_id": "UNKNOWN:0001",
  "gene": "UniProtKB:P56851",
  "gene_name": "Epididymal secretory protein E3-beta"
}